{
  "gene_symbol": "ANXA13",
  "term_id": "GO:0005737",
  "term_label": "cytoplasm",
  "gene_name": "Annexin A13",
  "gene": "UniProtKB:P27216"
}